{
  "term_label": "nucleus",
  "gene_symbol": "FHIT",
  "gene_name": "Bis(5'-adenosyl)-triphosphatase",
  "term_id": "GO:0005634",
  "gene": "UniProtKB:P49789"
}